abducens nerve structural organization [GO:0021600] (biological process) Also known as: abducens nerve structural organisation, CN VI structural organization Sources: GOC:cls, GOC:dgh, GOC:dph, GOC:jid, GO_REF:0000021 Definition: The process that contributes to the act of creating the structural organization of the abducens nerve. This process pertains to the physical shaping of a rudimentary structure. The motor function of the abducens nerve is to contract the lateral rectus which results in abduction of the eye. Relationships: is a type of cranial nerve structural organization [GO:0021604]; is part of abducens nerve morphogenesis [GO:0021598]